{
  "gene_name": "Transmembrane protein 114",
  "gene": "UniProtKB:B3SHH9",
  "term_label": "Unknown molecular function",
  "gene_symbol": "TMEM114",
  "term_id": "UNKNOWN:0001"
}